{
  "gene": "UniProtKB:Q8WY21",
  "term_label": "post-Golgi vesicle-mediated transport",
  "gene_symbol": "SORCS1",
  "term_id": "GO:0006892",
  "gene_name": "VPS10 domain-containing receptor SorCS1"
}